{
  "term_label": "positive regulation of cell population proliferation",
  "gene_symbol": "FGF19",
  "gene_name": "Fibroblast growth factor 19",
  "term_id": "GO:0008284",
  "gene": "UniProtKB:O95750"
}